{
  "gene_name": "Cytosolic carboxypeptidase 6",
  "term_label": "metallocarboxypeptidase activity",
  "gene_symbol": "AGBL4",
  "term_id": "GO:0004181",
  "gene": "UniProtKB:Q5VU57"
}